{
  "term_label": "intracellular protein localization",
  "term_id": "GO:0008104",
  "gene": "UniProtKB:P27348",
  "gene_name": "14-3-3 protein theta",
  "gene_symbol": "YWHAQ"
}